{
  "term_label": "nucleus",
  "gene_symbol": "FOXR2",
  "term_id": "GO:0005634",
  "gene": "UniProtKB:Q6PJQ5",
  "gene_name": "Forkhead box protein R2"
}